{
  "term_label": "pre-miRNA processing",
  "gene": "UniProtKB:Q9H9Z2",
  "gene_name": "Protein lin-28 homolog A",
  "term_id": "GO:0031054",
  "gene_symbol": "LIN28A"
}